beta-N-acetylglucosaminylglycopeptide beta-1,4-galactosyltransferase activity [GO:0003831] (molecular function) Also known as: thyroid galactosyltransferase activity, thyroid glycoprotein beta-galactosyltransferase, GalT activity, UDP-galactose--glycoprotein galactosyltransferase activity, UDP-galactose:N-acetyl-beta-D-glucosaminylglycopeptide beta-1,4-galactosyltransferase activity, UDPgalactose-glycoprotein galactosyltransferase activity, UDPgalactose:N-acetyl-beta-D-glucosaminylglycopeptide beta-1,4-galactosyltransferase activity, beta-N-acetyl-beta-(1,4)-galactosyltransferase activity, beta-N-acetyl-beta-1,4-galactosyltransferase activity, glycoprotein 4-beta-galactosyl-transferase activity, glycoprotein 4-beta-galactosyltransferase activity, glycoprotein beta-galactosyltransferase activity, uridine diphosphogalactose-glycoprotein galactosyltransferase activity Definition: Catalysis of the reaction: UDP-galactose + N-acetyl-beta-D-glucosaminylglycopeptide = UDP + beta-D-galactosyl-(1->4)-N-acetyl-beta-D-glucosaminylglycopeptide. Relationships: is a type of UDP-galactosyltransferase activity [GO:0035250] Sources: EC:2.4.1.38